{
  "gene_symbol": "KDM6B",
  "term_id": "GO:0031490",
  "gene": "UniProtKB:O15054",
  "gene_name": "Lysine-specific demethylase 6B",
  "term_label": "chromatin DNA binding"
}